{
  "gene": "UniProtKB:Q8WWX0",
  "gene_symbol": "ASB5",
  "gene_name": "Ankyrin repeat and SOCS box protein 5",
  "term_label": "Unknown cellular component",
  "term_id": "UNKNOWN:0003"
}